alpha-amino acid biosynthetic process [GO:1901607] (biological process) Subtypes: alanine biosynthetic process [GO:0006523], ornithine biosynthetic process [GO:0006592], serine family amino acid biosynthetic process [GO:0009070], isoleucine biosynthetic process [GO:0009097], citrulline biosynthetic process [GO:0019240], 4-hydroxyproline biosynthetic process [GO:0019472], 1-aminocyclopropane-1-carboxylate biosynthetic process [GO:0042218], D-amino acid biosynthetic process [GO:0046437], homocysteine biosynthetic process [GO:0071268], GO:0170034, GO:1901054 Sources: GOC:TermGenie Also known as: alpha-amino acid anabolism, alpha-amino acid biosynthesis, alpha-amino acid formation, alpha-amino acid synthesis Definition: The chemical reactions and pathways resulting in the formation of an alpha-amino acid. Relationships: is a type of GO:0008652; is a type of carboxylic acid biosynthetic process [GO:0046394]; is a type of alpha-amino acid metabolic process [GO:1901605]